{
  "gene_name": "Coiled-coil domain-containing protein 32",
  "term_id": "GO:0044782",
  "gene": "UniProtKB:Q9BV29",
  "gene_symbol": "CCDC32",
  "term_label": "cilium organization"
}